{
  "gene_symbol": "ACSM2A",
  "term_label": "fatty-acyl-CoA synthase activity",
  "term_id": "GO:0004321",
  "gene_name": "Acyl-coenzyme A synthetase ACSM2A, mitochondrial",
  "gene": "UniProtKB:Q08AH3"
}